{
  "gene": "UniProtKB:P54578",
  "gene_name": "Ubiquitin carboxyl-terminal hydrolase 14",
  "term_id": "GO:0070628",
  "term_label": "proteasome binding",
  "gene_symbol": "USP14"
}